{
  "term_id": "UNKNOWN:0001",
  "gene_name": "Ubiquitin carboxyl-terminal hydrolase 22",
  "term_label": "Unknown molecular function",
  "gene_symbol": "USP22",
  "gene": "UniProtKB:Q9UPT9"
}